{
  "gene": "UniProtKB:Q68CQ4",
  "gene_symbol": "UTP25",
  "term_label": "nucleolus",
  "gene_name": "U3 small nucleolar RNA-associated protein 25 homolog",
  "term_id": "GO:0005730"
}